poly-hydroxybutyrate metabolic process [GO:0042618] (biological process) Also known as: PHB metabolic process, PHB metabolism, poly-hydroxybutyrate metabolism Subtypes: poly-hydroxybutyrate biosynthetic process [GO:0042619] References: PMID:18640095 Sources: GOC:jl Relationships: is_a poly(hydroxyalkanoate) metabolic process [GO:1901440] Definition: The chemical reactions and pathways involving poly-hydroxybutyrate (PHB), a polymer of beta-hydroxybutyrate and a common storage material of prokaryotic cells.